{
  "term_id": "GO:0050911",
  "term_label": "detection of chemical stimulus involved in sensory perception of smell",
  "gene_symbol": "OR12D2",
  "gene": "UniProtKB:P58182",
  "gene_name": "Olfactory receptor 12D2"
}